{
  "term_label": "Unknown cellular component",
  "gene_symbol": "MYT1L",
  "gene": "UniProtKB:Q9UL68",
  "gene_name": "Myelin transcription factor 1-like protein",
  "term_id": "UNKNOWN:0003"
}